juxtaglomerular apparatus development [GO:0072051] (biological process) Subtypes: mesonephric juxtaglomerular apparatus development [GO:0061212], GO:0072206 Definition: The process whose specific outcome is the progression of the juxtaglomerular apparatus over time, from its formation to the mature structure. The juxtaglomerular apparatus is an anatomical structure that lies adjacent to the glomerulus and regulates kidney function. Sources: GOC:mtg_kidney_jan10 Relationships: is a type of anatomical structure development [GO:0048856]; is part of kidney development [GO:0001822]